{
  "gene_symbol": "OR6C65",
  "gene_name": "Olfactory receptor 6C65",
  "term_label": "plasma membrane",
  "gene": "UniProtKB:A6NJZ3",
  "term_id": "GO:0005886"
}